pattern specification involved in mesonephros development [GO:0061227] (biological process) Sources: GOC:mtg_kidney_jan10 Also known as: mesonephros pattern specification, mesonephros pattern formation Definition: Any developmental process that results in the creation of defined areas or spaces within the mesonephros to which cells respond and eventually are instructed to differentiate. Relationships: is a type of GO:0061004; is part of mesonephros development [GO:0001823] Subtypes: proximal/distal pattern formation involved in mesonephric nephron development [GO:0061226], specification of mesonephric nephron tubule identity [GO:0061282], GO:0061288, GO:0072099, GO:0072167